{
  "gene_symbol": "ARL15",
  "gene": "UniProtKB:Q9NXU5",
  "gene_name": "ADP-ribosylation factor-like protein 15",
  "term_label": "Unknown biological process",
  "term_id": "UNKNOWN:0002"
}